{
  "gene": "UniProtKB:Q8N1T3",
  "term_id": "GO:0015629",
  "term_label": "actin cytoskeleton",
  "gene_symbol": "MYO1H",
  "gene_name": "Unconventional myosin-Ih"
}